isopentenyl phosphate kinase activity [GO:0102043] (MF) References: PMID:19928876 Sources: GOC:pz, RHEA:33963 Relationships: is a type of GO:0016776 Definition: Catalysis of the reaction: isopentenyl phosphate(2-) + ATP(4-) = isopentenyl diphosphate(3-) + ADP(3-).